{
  "gene": "UniProtKB:P00519",
  "gene_name": "Tyrosine-protein kinase ABL1",
  "term_label": "positive regulation of endothelial cell migration",
  "gene_symbol": "ABL1",
  "term_id": "GO:0010595"
}